{
  "term_label": "cullin family protein binding",
  "term_id": "GO:0097602",
  "gene": "UniProtKB:Q9NYG5",
  "gene_name": "Anaphase-promoting complex subunit 11",
  "gene_symbol": "ANAPC11"
}